{
  "term_id": "GO:0045892",
  "gene": "UniProtKB:Q15834",
  "term_label": "negative regulation of DNA-templated transcription",
  "gene_symbol": "CCDC85B",
  "gene_name": "Coiled-coil domain-containing protein 85B"
}